{
  "gene": "UniProtKB:P07900",
  "gene_name": "Heat shock protein HSP 90-alpha",
  "term_label": "protein stabilization",
  "gene_symbol": "HSP90AA1",
  "term_id": "GO:0050821"
}